{
  "gene_name": "Transmembrane ascorbate-dependent reductase CYB561",
  "term_label": "Unknown biological process",
  "term_id": "UNKNOWN:0002",
  "gene_symbol": "CYB561",
  "gene": "UniProtKB:P49447"
}